{
  "gene_name": "CUGBP Elav-like family member 4",
  "gene": "UniProtKB:Q9BZC1",
  "gene_symbol": "CELF4",
  "term_id": "GO:0005737",
  "term_label": "cytoplasm"
}